{
  "term_id": "UNKNOWN:0003",
  "term_label": "Unknown cellular component",
  "gene": "UniProtKB:O75891",
  "gene_name": "Cytosolic 10-formyltetrahydrofolate dehydrogenase",
  "gene_symbol": "ALDH1L1"
}